{
  "term_label": "odorant binding",
  "gene_symbol": "OR5B17",
  "term_id": "GO:0005549",
  "gene_name": "Olfactory receptor 5B17",
  "gene": "UniProtKB:Q8NGF7"
}